iridosome [GO:0043698] (cellular component) Sources: GOC:mh Definition: A tissue-specific, membrane-bounded cytoplasmic organelle within which purines crystalize in reflective stacks. Iridosomes are synthesized in iridophore cells and are silver, gold or iridescent in appearance. Relationships: is_a pigment granule [GO:0048770] Also known as: reflecting platelet